stellate cell precursor proliferation [GO:0021929] (biological process) References: PMID:15157725 Sources: GOC:cls, GOC:dgh, GOC:dph, GOC:jid, GO_REF:0000021 Relationships: is a type of cell proliferation in hindbrain ventricular zone [GO:0021923] Definition: The multiplication or reproduction of neuroblasts that will give rise to stellate cells. A cerebellar stellate cell is an inhibitory GABAergic interneuron found in the cerebellar cortex.